{
  "term_label": "ferric-chelate reductase (NADPH) activity",
  "gene_name": "Metalloreductase STEAP4",
  "term_id": "GO:0052851",
  "gene": "UniProtKB:Q687X5",
  "gene_symbol": "STEAP4"
}